styrene metabolic process [GO:0018966] (biological process) Definition: The chemical reactions and pathways involving styrene, an aromatic hydrocarbon liquid soluble in ether and alcohol. When heated, exposed to light or added to a peroxide catalyst, it undergoes polymerization to form polystyrene, a versatile material used in the manufacture of plastics, synthetic rubber, thermal insulation, and packaging. Styrene is a classified mutagen and a suspected carcinogen. Sources: GOC:jl, UM-BBD_pathwayID:sty Also known as: styrene metabolism Relationships: is a type of benzene-containing compound metabolic process [GO:0042537]; is a type of hydrocarbon metabolic process [GO:0120252]; is a type of olefinic compound metabolic process [GO:0120254] Subtypes: GO:0042207